CD20-Lck-Lyn-Fyn complex [GO:0070332] (cellular component) Definition: A protein complex that contains the cell-surface protein CD20 and the Src family tyrosine kinases Lck, Lyn and Fyn. References: PMID:7545683 Sources: GOC:mah Relationships: is a type of intracellular protein-containing complex [GO:0140535]; is a type of catalytic complex [GO:1902494]